regulation of keratinocyte proliferation [GO:0010837] (biological process) Definition: Any process that modulates the rate, frequency or extent of keratinocyte proliferation. Keratinocyte proliferation is the multiplication or reproduction of keratinocytes, resulting in the expansion of a cell population. Sources: GOC:dph, GOC:tb Relationships: is a type of regulation of epithelial cell proliferation [GO:0050678]; regulates GO:0043616 Subtypes: positive regulation of keratinocyte proliferation [GO:0010838], negative regulation of keratinocyte proliferation [GO:0010839]